{
  "term_label": "L-histidine transmembrane transporter activity",
  "term_id": "GO:0005290",
  "gene": "UniProtKB:Q8N697",
  "gene_name": "Solute carrier family 15 member 4",
  "gene_symbol": "SLC15A4"
}